{
  "gene_symbol": "CT55",
  "gene_name": "Cancer_testis antigen 55",
  "term_label": "Unknown biological process",
  "term_id": "UNKNOWN:0002",
  "gene": "UniProtKB:Q8WUE5"
}